{
  "gene": "UniProtKB:Q86XT4",
  "term_id": "GO:0045087",
  "term_label": "innate immune response",
  "gene_symbol": "TRIM50",
  "gene_name": "E3 ubiquitin-protein ligase TRIM50"
}